Cry-Per complex [GO:1990512] (cellular component) Definition: Nuclear transcriptional repressor complex that is capable of negatively regulating CLOCK-BMAL-dependent transactivation of genes in a delayed negative feedback manner which generates circadian rhythms. Relationships: is a type of transcription repressor complex [GO:0017053]; is a type of nuclear protein-containing complex [GO:0140513] Note: An example of this is Cry1 in mouse (P97784) in PMID:24855952 (inferred from physical interaction). References: PMID:24855952 Sources: GOC:bhm